{
  "gene_name": "Cytochrome c oxidase subunit 2",
  "gene_symbol": "MT-CO2",
  "gene": "UniProtKB:P00403",
  "term_label": "respiratory chain complex IV",
  "term_id": "GO:0045277"
}